{
  "gene_name": "Ras association domain-containing protein 10",
  "gene": "UniProtKB:A6NK89",
  "gene_symbol": "RASSF10",
  "term_id": "UNKNOWN:0003",
  "term_label": "Unknown cellular component"
}